{
  "term_label": "DNA binding",
  "gene_name": "Meiotic recombination protein SPO11",
  "gene_symbol": "SPO11",
  "term_id": "GO:0003677",
  "gene": "UniProtKB:Q9Y5K1"
}